negative regulation of chloride transport [GO:2001226] (biological process) Sources: GOC:dph Definition: Any process that stops, prevents or reduces the frequency, rate or extent of chloride transport. Relationships: is a type of GO:1903792; is a type of regulation of chloride transport [GO:2001225]; negatively regulates GO:0006821